{
  "gene": "UniProtKB:Q9NYY3",
  "gene_symbol": "PLK2",
  "term_id": "GO:0000776",
  "gene_name": "Serine_threonine-protein kinase PLK2",
  "term_label": "kinetochore"
}